spermidine:coumaroyl CoA N-acyltransferase activity [GO:0080073] (molecular function) Definition: Catalysis of the transfer of a coumaroyl group to a nitrogen atom on the spermidine molecule. Relationships: is a type of N-acyltransferase activity [GO:0016410] References: PMID:19077165